formimidoyltetrahydrofolate cyclodeaminase activity [GO:0030412] (molecular function) Note: Note that cyclodeaminases are lyases according to EC, whereas deaminases are hydrolases. Relationships: is a type of GO:0016841 Also known as: 5-formimidoyltetrahydrofolate ammonia-lyase (cyclizing), 5-formimidoyltetrahydrofolate ammonia-lyase (cyclizing; 5,10-methenyltetrahydrofolate-forming), formiminotetrahydrofolate cyclodeaminase activity Definition: Catalysis of the reaction: 5-formimidoyltetrahydrofolate + 2 H+ = 5,10-methenyltetrahydrofolate + NH4. Sources: EC:4.3.1.4, RHEA:22736